{
  "term_id": "GO:0005634",
  "term_label": "nucleus",
  "gene_symbol": "NEUROD1",
  "gene": "UniProtKB:Q13562",
  "gene_name": "Neurogenic differentiation factor 1"
}